{
  "gene": "UniProtKB:O75973",
  "gene_symbol": "C1QL1",
  "term_id": "GO:0099550",
  "term_label": "trans-synaptic signaling, modulating synaptic transmission",
  "gene_name": "C1q-related factor"
}